{
  "term_label": "endoplasmic reticulum membrane",
  "gene_name": "Reticulon-2",
  "gene_symbol": "RTN2",
  "term_id": "GO:0005789",
  "gene": "UniProtKB:O75298"
}